deoxyribonucleoside biosynthetic process [GO:0046120] (biological process) Subtypes: GO:0046123, pyrimidine deoxyribonucleoside biosynthetic process [GO:0046126] Definition: The chemical reactions and pathways resulting in the formation of any one of a family of organic molecules consisting of a purine or pyrimidine base covalently bonded to a sugar deoxyribose (a deoxyribonucleoside). Relationships: is a type of GO:0009120; is_a nucleoside biosynthetic process [GO:0009163] Also known as: deoxyribonucleoside anabolism, deoxyribonucleoside biosynthesis, deoxyribonucleoside formation, deoxyribonucleoside synthesis Sources: GOC:ai